{
  "gene_name": "Small ribosomal subunit protein uS12m",
  "term_id": "GO:0003735",
  "gene_symbol": "MRPS12",
  "term_label": "structural constituent of ribosome",
  "gene": "UniProtKB:O15235"
}